{
  "term_label": "Unknown molecular function",
  "term_id": "UNKNOWN:0001",
  "gene": "UniProtKB:Q5VUB5",
  "gene_symbol": "FAM171A1",
  "gene_name": "Protein FAM171A1"
}